{
  "term_id": "UNKNOWN:0001",
  "gene_name": "E3 ubiquitin-protein ligase RNF187",
  "term_label": "Unknown molecular function",
  "gene_symbol": "RNF187",
  "gene": "UniProtKB:Q5TA31"
}